{
  "gene_symbol": "FAM83E",
  "gene_name": "Protein FAM83E",
  "gene": "UniProtKB:Q2M2I3",
  "term_label": "protein kinase binding",
  "term_id": "GO:0019901"
}